lncRNA binding [GO:0106222] (molecular function) Also known as: long noncoding RNA binding Definition: Binding to a long noncoding RNA (lncRNA). References: PMID:25578728 Relationships: is a type of RNA binding [GO:0003723]